primary cell septum [GO:0000936] (cellular component) Definition: A cell septum that forms following nuclear division. Sources: GOC:clt, ISBN:0471940526 Also known as: primary septum Relationships: is a type of GO:0000935